{
  "gene": "UniProtKB:P52198",
  "term_label": "regulation of actin cytoskeleton organization",
  "gene_symbol": "RND2",
  "term_id": "GO:0032956",
  "gene_name": "Rho-related GTP-binding protein RhoN"
}